{
  "gene": "UniProtKB:P54920",
  "gene_name": "Alpha-soluble NSF attachment protein",
  "term_id": "GO:0006886",
  "term_label": "intracellular protein transport",
  "gene_symbol": "NAPA"
}